negative regulation of short-term synaptic potentiation [GO:1905513] (biological process) Relationships: is a type of negative regulation of biological process [GO:0048519]; is a type of regulation of short-term synaptic potentiation [GO:1905512]; negatively regulates short-term synaptic potentiation [GO:1990926] References: PMID:15470145 Sources: GOC:TermGenie, GOC:hjd, GO_REF:0000058 Also known as: down regulation of short-term synaptic potentiation, down regulation of synaptic facilitation, down-regulation of short-term synaptic potentiation, down-regulation of synaptic facilitation, downregulation of short-term synaptic potentiation, downregulation of synaptic facilitation, negative regulation of synaptic facilitation, inhibition of short-term synaptic potentiation, inhibition of synaptic facilitation Definition: Any process that stops, prevents or reduces the frequency, rate or extent of short-term synaptic potentiation.